actin filament fragmentation [GO:0030043] (biological process) Sources: GOC:mah, ISBN:0815316194 Relationships: is a type of actin filament depolymerization [GO:0030042] Definition: The severing of actin filaments into numerous short fragments, usually mediated by actin severing proteins.